{
  "term_id": "GO:0046513",
  "term_label": "ceramide biosynthetic process",
  "gene_name": "Ceramide synthase 4",
  "gene_symbol": "CERS4",
  "gene": "UniProtKB:Q9HA82"
}